{
  "gene_symbol": "OR1L3",
  "term_id": "GO:0004984",
  "term_label": "olfactory receptor activity",
  "gene_name": "Olfactory receptor 1L3",
  "gene": "UniProtKB:Q8NH93"
}